phosphoribosyl-AMP cyclohydrolase activity [GO:0004635] (molecular function) Definition: Catalysis of the reaction: 1-(5-phosphonatoribosyl)-5'-AMP + H2O = 1-(5-phosphoribosyl)-5-[(5-phosphoribosylamino)methylideneamino]imidazole-4-carboxamide. Sources: EC:3.5.4.19, RHEA:20049 Also known as: 1-(5-phospho-D-ribosyl)-AMP 1,6-hydrolase activity, PRAMP-cyclohydrolase activity, phosphoribosyladenosine monophosphate cyclohydrolase activity Relationships: is a type of GO:0019238